{
  "term_id": "GO:0005635",
  "gene_symbol": "PLA2G4C",
  "gene_name": "Cytosolic phospholipase A2 gamma",
  "gene": "UniProtKB:Q9UP65",
  "term_label": "nuclear envelope"
}